L-methionine (R)-S-oxide reductase activity [GO:0033745] (molecular function) Relationships: is a type of oxidoreductase activity, acting on a sulfur group of donors, disulfide as acceptor [GO:0016671] Also known as: FRMsr, L-methionine:thioredoxin-disulfide S-oxidoreductase [L-methionine (R)-S-oxide-forming] activity, free met-R-(o) reductase activity, free-methionine (R)-S-oxide reductase activity, methionine-R-sulfoxide reductase activity Sources: RHEA:21260 Definition: Catalysis of the reaction: [thioredoxin]-disulfide + L-methionine + H2O = L-methionine (R)-S-oxide + [thioredoxin]-dithiol.